{
  "term_label": "Unknown cellular component",
  "gene_name": "Coiled-coil domain-containing glutamate-rich protein 2",
  "term_id": "UNKNOWN:0003",
  "gene_symbol": "CCER2",
  "gene": "UniProtKB:I3L3R5"
}